{
  "gene_name": "Alpha-internexin",
  "gene_symbol": "INA",
  "term_id": "GO:0005882",
  "term_label": "intermediate filament",
  "gene": "UniProtKB:Q16352"
}